H-gal-GP complex [GO:1990850] (CC) Definition: A membrane glycoprotein complex with aspartyl proteinase and metalloproteinase activity which is expressed in the gut. An example of this is found in the nematode Haemonchus contortus. Also known as: Haemonchus galactose-containing glycoprotein complex, galactose-containing glycoprotein complex Relationships: is a type of GO:0098796; is a type of peptidase complex [GO:1905368] References: PMID:11166393